cellular developmental process [GO:0048869] (biological process) Relationships: is a type of cellular process [GO:0009987]; is a type of developmental process [GO:0032502] Subtypes: cell fate specification [GO:0001708], cell fate determination [GO:0001709], pre-B cell receptor expression [GO:0002330], donor selection [GO:0007535], GO:0009847, stomatal lineage progression [GO:0010440], programmed cell death involved in cell development [GO:0010623], initiation of movement involved in cerebral cortex radial glia guided migration [GO:0021806], cell differentiation [GO:0030154], centrosomal and pronuclear rotation [GO:0035047], heterocyst development [GO:0043158], cell dedifferentiation [GO:0043697], cell fate commitment [GO:0045165], GO:0048236, cell development [GO:0048468], cell maturation [GO:0048469], ascospore release from ascus [GO:0071998], cortical rotation [GO:0160174] Definition: A biological process whose specific outcome is the progression of a cell over time from an initial condition to a later condition. Sources: GOC:isa_complete